BBSome binding [GO:0062063] (molecular function) Definition: Binding to a BBSome complex. References: PMID:20603001 Relationships: is a type of protein-containing complex binding [GO:0044877]